nitrite reductase complex [NAD(P)H] [GO:0009344] (cellular component) Definition: Complex that possesses nitrite reductase [NAD(P)H] activity. Relationships: is a type of catalytic complex [GO:1902494] Note: See also the molecular function term 'nitrite reductase [NAD(P)H] activity ; GO:0008942'. Sources: GOC:mah